nerve growth factor receptor activity [GO:0010465] (molecular function) Definition: Combining with nerve growth factor (NGF), to prevent apoptosis in neurons and promote nerve growth, or to initiate a change in cell activity. Sources: GOC:dph, GOC:tb Also known as: NGF receptor activity, beta-nerve growth factor receptor activity Relationships: is a type of neurotrophin receptor activity [GO:0005030]; is part of nerve growth factor signaling pathway [GO:0038180]; has part nerve growth factor binding [GO:0048406] Regulation: RO_0002211 by GO:0051394